{
  "gene_symbol": "RNASE13",
  "gene": "UniProtKB:Q5GAN3",
  "term_label": "defense response to Gram-positive bacterium",
  "term_id": "GO:0050830",
  "gene_name": "Probable inactive ribonuclease-like protein 13"
}